{
  "gene_symbol": "MAML1",
  "gene_name": "Mastermind-like protein 1",
  "gene": "UniProtKB:Q92585",
  "term_id": "GO:0003713",
  "term_label": "transcription coactivator activity"
}